{
  "term_id": "GO:0004435",
  "term_label": "phosphatidylinositol-4,5-bisphosphate phospholipase C activity",
  "gene_name": "1-phosphatidylinositol 4,5-bisphosphate phosphodiesterase eta-2",
  "gene_symbol": "PLCH2",
  "gene": "UniProtKB:O75038"
}